response to polycyclic arene [GO:1903165] (biological process) References: PMID:10998501 Sources: GOC:TermGenie, GOC:mr, GO_REF:0000071 Definition: Any process that results in a change in state or activity of a cell or an organism (in terms of movement, secretion, enzyme production, gene expression, etc.) as a result of a polycyclic arene stimulus. Relationships: is a type of response to chemical [GO:0042221] Subtypes: cellular response to polycyclic arene [GO:1903166], response to 3-methylcholanthrene [GO:1904681]